{
  "term_label": "Unknown molecular function",
  "gene_name": "Trafficking protein particle complex subunit 2B",
  "gene": "UniProtKB:P0DI82",
  "gene_symbol": "TRAPPC2B",
  "term_id": "UNKNOWN:0001"
}